{
  "gene": "UniProtKB:P80748",
  "gene_name": "Immunoglobulin lambda variable 3-21",
  "gene_symbol": "IGLV3-21",
  "term_label": "immunoglobulin complex",
  "term_id": "GO:0019814"
}